{
  "gene_symbol": "HSFX4",
  "gene": "UniProtKB:A0A1B0GTS1",
  "gene_name": "Heat shock transcription factor, X-linked member 4",
  "term_id": "GO:0003700",
  "term_label": "DNA-binding transcription factor activity"
}